{
  "gene": "UniProtKB:Q9Y2G4",
  "gene_name": "Ankyrin repeat domain-containing protein 6",
  "gene_symbol": "ANKRD6",
  "term_id": "GO:0030111",
  "term_label": "regulation of Wnt signaling pathway"
}